positive regulation of peptide antigen transport [GO:1901041] (biological process) Relationships: is a type of GO:0002585; is a type of positive regulation of transport [GO:0051050]; is a type of regulation of peptide antigen transport [GO:1901039]; RO_0002213 peptide antigen transport [GO:0046968] Sources: GOC:TermGenie, GOC:bf Definition: Any process that activates or increases the frequency, rate or extent of peptide antigen transport. Also known as: up regulation of peptide antigen transport, up-regulation of peptide antigen transport, upregulation of peptide antigen transport, activation of peptide antigen transport